{
  "gene_name": "Sodium_calcium exchanger 2",
  "term_id": "GO:1990034",
  "gene_symbol": "SLC8A2",
  "gene": "UniProtKB:Q9UPR5",
  "term_label": "calcium ion export across plasma membrane"
}